{
  "term_label": "Unknown molecular function",
  "term_id": "UNKNOWN:0001",
  "gene": "UniProtKB:O75935",
  "gene_name": "Dynactin subunit 3",
  "gene_symbol": "DCTN3"
}